{
  "gene_name": "Tax1-binding protein 3",
  "gene": "UniProtKB:O14907",
  "term_id": "UNKNOWN:0003",
  "term_label": "Unknown cellular component",
  "gene_symbol": "TAX1BP3"
}